{
  "gene_symbol": "INO80",
  "gene_name": "Chromatin-remodeling ATPase INO80",
  "term_id": "GO:0042393",
  "term_label": "histone binding",
  "gene": "UniProtKB:Q9ULG1"
}